dopaminergic neuron differentiation [GO:0071542] (biological process) Subtypes: GO:1904948 Definition: The process in which a neuroblast acquires the specialized structural and functional features of a dopaminergic neuron, a neuron that secretes dopamine. Regulation: regulated by regulation of dopaminergic neuron differentiation [GO:1904338]; negatively regulated by negative regulation of dopaminergic neuron differentiation [GO:1904339]; positively regulated by positive regulation of dopaminergic neuron differentiation [GO:1904340] Relationships: is a type of GO:0030182 Sources: GOC:rph